{
  "gene": "UniProtKB:Q13507",
  "term_id": "GO:0015279",
  "gene_symbol": "TRPC3",
  "gene_name": "Short transient receptor potential channel 3",
  "term_label": "store-operated calcium channel activity"
}